{
  "gene_name": "DNA-directed RNA polymerase III subunit RPC4",
  "term_id": "UNKNOWN:0001",
  "gene": "UniProtKB:P05423",
  "term_label": "Unknown molecular function",
  "gene_symbol": "POLR3D"
}